{
  "term_id": "GO:0070098",
  "gene": "UniProtKB:P55773",
  "term_label": "chemokine-mediated signaling pathway",
  "gene_symbol": "CCL23",
  "gene_name": "C-C motif chemokine 23"
}